{
  "gene_symbol": "SCMH1",
  "gene_name": "Polycomb protein SCMH1",
  "term_label": "negative regulation of DNA-templated transcription",
  "term_id": "GO:0045892",
  "gene": "UniProtKB:Q96GD3"
}